pyrimidine ribonucleoside monophosphate catabolic process [GO:0009175] (biological process) Definition: The chemical reactions and pathways resulting in the breakdown of pyrimidine ribonucleoside monophosphate, a compound consisting of a pyrimidine base linked to a ribose sugar esterified with phosphate on the sugar. Also known as: pyrimidine ribonucleoside monophosphate breakdown, pyrimidine ribonucleoside monophosphate catabolism, pyrimidine ribonucleoside monophosphate degradation Relationships: is a type of pyrimidine nucleoside monophosphate catabolic process [GO:0009131]; is a type of ribonucleoside monophosphate catabolic process [GO:0009158]; is a type of pyrimidine ribonucleoside monophosphate metabolic process [GO:0009173] Subtypes: CMP catabolic process [GO:0006248], TMP catabolic process [GO:0046045], GO:0046050 Sources: GOC:go_curators, ISBN:0198506732